{
  "gene": "UniProtKB:Q8IVK1",
  "term_label": "Unknown cellular component",
  "term_id": "UNKNOWN:0003",
  "gene_symbol": "GLYCAM1",
  "gene_name": "Putative glycosylation-dependent cell adhesion molecule 1"
}